{
  "term_label": "removal of superoxide radicals",
  "gene_symbol": "CCS",
  "term_id": "GO:0019430",
  "gene_name": "Copper chaperone for superoxide dismutase",
  "gene": "UniProtKB:O14618"
}